hydrogen:quinone oxidoreductase activity [GO:0047067] (molecular function) Sources: EC:1.12.5.1, RHEA:18641 Also known as: membrane-bound hydrogenase activity, hydrogen-ubiquinone oxidoreductase activity, hydrogen:menaquinone oxidoreductase activity, quinone-reactive Ni/Fe-hydrogenase activity Definition: Catalysis of the reaction: H(2) + menaquinone = reduced menaquinone. Relationships: is a type of oxidoreductase activity, acting on hydrogen as donor, with a quinone or similar compound as acceptor [GO:0046994]